{
  "gene_name": "Zinc finger protein 695",
  "term_label": "regulation of DNA-templated transcription",
  "gene": "UniProtKB:Q8IW36",
  "gene_symbol": "ZNF695",
  "term_id": "GO:0006355"
}